phosphate ion transport [GO:0006817] (biological process) Relationships: is a type of inorganic anion transport [GO:0015698] Regulation: regulated by GO:0010966 Sources: GOC:krc Subtypes: GO:0035435, sodium-dependent phosphate transport [GO:0044341] Definition: The directed movement of phosphate ions into, out of or within a cell, or between cells, by means of some agent such as a transporter or pore. Also known as: phosphate transport